{
  "gene": "UniProtKB:A6NM28",
  "term_id": "GO:0005634",
  "term_label": "nucleus",
  "gene_symbol": "ZFP92",
  "gene_name": "Zinc finger protein 92 homolog"
}